{
  "gene": "UniProtKB:O14610",
  "gene_name": "Guanine nucleotide-binding protein G(I)_G(S)_G(O) subunit gamma-T2",
  "term_id": "GO:0007186",
  "term_label": "G protein-coupled receptor signaling pathway",
  "gene_symbol": "GNGT2"
}